{
  "term_label": "G protein-coupled receptor kinase activity",
  "gene_symbol": "GRK2",
  "gene_name": "Beta-adrenergic receptor kinase 1",
  "gene": "UniProtKB:P25098",
  "term_id": "GO:0004703"
}